L-phenylalanine biosynthetic process [GO:0009094] (biological process) Relationships: is a type of L-phenylalanine metabolic process [GO:0006558]; is a type of aromatic amino acid family biosynthetic process, prephenate pathway [GO:0009095]; is a type of GO:0170034; is a type of proteinogenic amino acid biosynthetic process [GO:0170038] Definition: The chemical reactions and pathways resulting in the formation of L-phenylalanine, the L-enantiomer of 2-amino-3-phenylpropanoic acid, i.e. (2S)-2-amino-3-phenylpropanoic acid. Also known as: phenylalanine biosynthesis, phenylalanine biosynthetic process, L-phenylalanine anabolism, L-phenylalanine biosynthesis, L-phenylalanine formation, L-phenylalanine synthesis, phenylalanine biosynthetic process, prephenate pathway, phenylalanine biosynthetic process, shikimate pathway Sources: GOC:jsg, GOC:mah Subtypes: L-phenylalanine biosynthetic process from chorismate via phenylpyruvate [GO:0033585], L-phenylalanine biosynthetic process from chorismate via L-arogenate [GO:0033586]